{
  "term_id": "UNKNOWN:0001",
  "gene": "UniProtKB:Q9NZV1",
  "gene_name": "Cysteine-rich motor neuron 1 protein",
  "gene_symbol": "CRIM1",
  "term_label": "Unknown molecular function"
}